negative regulation of brown fat cell proliferation [GO:0070348] (biological process) Also known as: down regulation of brown fat cell proliferation, down-regulation of brown fat cell proliferation, downregulation of brown fat cell proliferation, negative regulation of brown adipocyte proliferation, negative regulation of brown adipose cell proliferation, inhibition of brown fat cell proliferation Sources: GOC:mah, GOC:sl Definition: Any process that stops or decreases the rate or extent of brown fat cell proliferation. Relationships: is a type of negative regulation of fat cell proliferation [GO:0070345]; is a type of regulation of brown fat cell proliferation [GO:0070347]; negatively regulates brown fat cell proliferation [GO:0070342]